regulation of transforming growth factor beta3 production [GO:0032910] (biological process) Sources: GOC:mah Definition: Any process that modulates the frequency, rate, or extent of production of transforming growth factor-beta3. Also known as: regulation of TGF-B3 production, regulation of TGFB3 production, regulation of transforming growth factor-beta3 production Subtypes: negative regulation of transforming growth factor beta3 production [GO:0032913], GO:0032916 Relationships: is a type of GO:0071634; regulates GO:0032907